{
  "gene_name": "Interferon alpha-inducible protein 27-like protein 1",
  "gene": "UniProtKB:Q96BM0",
  "gene_symbol": "IFI27L1",
  "term_label": "molecular adaptor activity",
  "term_id": "GO:0060090"
}